{
  "gene_name": "Adenylyltransferase and sulfurtransferase MOCS3",
  "gene": "UniProtKB:O95396",
  "term_id": "GO:0016779",
  "gene_symbol": "MOCS3",
  "term_label": "nucleotidyltransferase activity"
}